{
  "gene": "UniProtKB:Q8NAT2",
  "gene_symbol": "TDRD5",
  "term_id": "UNKNOWN:0003",
  "term_label": "Unknown cellular component",
  "gene_name": "Tudor domain-containing protein 5"
}